transporter activator activity [GO:0141109] (molecular function) Relationships: is a type of molecular function activator activity [GO:0140677]; is a type of transporter regulator activity [GO:0141108]; positively regulates GO:0005215 Subtypes: channel activator activity [GO:0099103] Sources: GOC:curators Definition: Binds to and increases the activity of a transporter.